{
  "gene_symbol": "GATA1",
  "gene_name": "Erythroid transcription factor",
  "gene": "UniProtKB:P15976",
  "term_id": "GO:0045165",
  "term_label": "cell fate commitment"
}